{
  "term_label": "DNA binding",
  "term_id": "GO:0003677",
  "gene_name": "Tigger transposable element-derived protein 2",
  "gene": "UniProtKB:Q4W5G0",
  "gene_symbol": "TIGD2"
}